{
  "gene_symbol": "IRF8",
  "term_id": "GO:0005634",
  "term_label": "nucleus",
  "gene": "UniProtKB:Q02556",
  "gene_name": "Interferon regulatory factor 8"
}